phosphotransferase activity, alcohol group as acceptor [GO:0016773] (molecular function) Subtypes: GO:0000215, NAD+ kinase activity [GO:0003951], adenylylsulfate kinase activity [GO:0004020], choline kinase activity [GO:0004103], dephospho-CoA kinase activity [GO:0004140], GO:0004143, GO:0004168, ethanolamine kinase activity [GO:0004305], GO:0004335, GO:0004370, glycerone kinase activity [GO:0004371], GO:0004396, homoserine kinase activity [GO:0004413], GO:0004417, GO:0004454, mevalonate kinase activity [GO:0004496], GO:0004594, protein kinase activity [GO:0004672], pyruvate kinase activity [GO:0004743], ribokinase activity [GO:0004747], shikimate kinase activity [GO:0004765], D-xylulokinase activity [GO:0004856], GO:0008443, pyridoxal kinase activity [GO:0008478], GO:0008481, riboflavin kinase activity [GO:0008531], 2-dehydro-3-deoxygalactonokinase activity [GO:0008671], 2-dehydro-3-deoxygluconokinase activity [GO:0008673], GO:0008737, ribulokinase activity [GO:0008741], glycerate kinase activity [GO:0008887], GO:0008902, inosine kinase activity [GO:0008906], phosphoribulokinase activity [GO:0008974], protein-N(PI)-phosphohistidine-sugar phosphotransferase activity [GO:0008982], rhamnulokinase activity [GO:0008993], tagatose-6-phosphate kinase activity [GO:0009024], GO:0009029, undecaprenol kinase activity [GO:0009038], N-acylmannosamine kinase activity [GO:0009384], GO:0009702, phenol kinase activity [GO:0018720], inositol 3-kinase activity [GO:0019140], D-ribulokinase activity [GO:0019150], GO:0019165, GO:0019206, N-acetylgalactosamine kinase activity [GO:0033858], aminoglycoside phosphotransferase activity [GO:0034071], NADH kinase activity [GO:0042736], LPPG:FO 2-phospho-L-lactate transferase activity [GO:0043743], adenosylcobinamide kinase activity [GO:0043752], GO:0043798, GO:0043843, ADP-specific phosphofructokinase activity [GO:0043844], phosphoserine:homoserine phosphotransferase activity [GO:0043899], L-seryl-tRNA(Sec) kinase activity [GO:0043915], phosphocholine transferase activity [GO:0044605], gluconokinase activity [GO:0046316], S-methyl-5-thioribose kinase activity [GO:0046522], diphosphate-protein phosphotransferase activity [GO:0047321], GO:0047324, glycerol-3-phosphate-glucose phosphotransferase activity [GO:0047327], acyl-phosphate-hexose phosphotransferase activity [GO:0047328], phosphoramidate-hexose phosphotransferase activity [GO:0047329], GO:0047330, diphosphate-glycerol phosphotransferase activity [GO:0047331], diphosphate-serine phosphotransferase activity [GO:0047332], 5-dehydro-2-deoxygluconokinase activity [GO:0047590], acylglycerol kinase activity [GO:0047620], GO:0047628, alkylglycerol kinase activity [GO:0047649], GO:0047650, AMP-thymidine kinase activity [GO:0047667], beta-glucoside kinase activity [GO:0047700], GO:0047814, GO:0047841, erythritol kinase activity [GO:0047878], GO:0047912, glucosamine kinase activity [GO:0047931], glucose-1,6-bisphosphate synthase activity [GO:0047933], GO:0047937, glucuronokinase activity [GO:0047940], hamamelose kinase activity [GO:0047976], GO:0047992, macrolide 2'-kinase activity [GO:0050073], nucleoside phosphotransferase activity [GO:0050146], GO:0050165, GO:0050190, phosphoribokinase activity [GO:0050195], GO:0050201, pseudouridine kinase activity [GO:0050225], riboflavin phosphotransferase activity [GO:0050257], ribosylnicotinamide kinase activity [GO:0050262], scyllo-inosamine 4-kinase activity [GO:0050276], GO:0050277, GO:0050317, triokinase activity [GO:0050354], viomycin kinase activity [GO:0050394], GO:0050400, 4-(cytidine 5'-diphospho)-2-C-methyl-D-erythritol kinase activity [GO:0050515], GO:0051731, GO:0051765, inositol trisphosphate kinase activity [GO:0051766], prenol kinase activity [GO:0052673], phosphatidylinositol kinase activity [GO:0052742], GO:0052836, diphosphoinositol tetrakisphosphate kinase activity [GO:0052839], GO:0061594, nicotinate riboside kinase activity [GO:0061769], protein-phosphocysteine-sugar phosphotransferase activity [GO:0090563], adenylylselenate kinase activity [GO:0098617], seryl-selenocysteinyl-tRNA kinase activity [GO:0098620], GO:0102193, inositol phosphorylceramide synthase activity [GO:0102770], GO:0103020, protein-N(pi)-phosphohistidine--N-acetyl-D-glucosamine phosphotransferase activity [GO:0103111], inositol pentakisphosphate kinase activity [GO:0120517], GO:0141035 Definition: Catalysis of the transfer of a phosphorus-containing group from one compound (donor) to an alcohol group (acceptor). Sources: EC:2.7.1.- Relationships: is a type of GO:0016772